{
  "term_label": "mitochondrion",
  "gene_symbol": "LDHAL6A",
  "gene_name": "L-lactate dehydrogenase A-like 6A",
  "term_id": "GO:0005739",
  "gene": "UniProtKB:Q6ZMR3"
}